{
  "gene": "UniProtKB:Q8N4L2",
  "gene_name": "Type 2 phosphatidylinositol 4,5-bisphosphate 4-phosphatase",
  "gene_symbol": "PIP4P2",
  "term_label": "lysosomal membrane",
  "term_id": "GO:0005765"
}